{
  "gene_symbol": "HAPLN1",
  "term_label": "perineuronal net",
  "gene_name": "Hyaluronan and proteoglycan link protein 1",
  "gene": "UniProtKB:P10915",
  "term_id": "GO:0072534"
}